{
  "gene": "UniProtKB:Q96DV4",
  "gene_symbol": "MRPL38",
  "term_id": "GO:0005762",
  "gene_name": "Large ribosomal subunit protein mL38",
  "term_label": "mitochondrial large ribosomal subunit"
}